choline monooxygenase activity [GO:0019133] (molecular function) Definition: Catalysis of the reaction: choline + 2 reduced ferredoxin + O2 + 2 H+ = betaine aldehyde hydrate + 2 oxidized ferredoxin + H2O. Sources: EC:1.14.15.7 Also known as: choline,reduced-ferredoxin:oxygen oxidoreductase activity Relationships: is a type of oxidoreductase activity, acting on paired donors, with incorporation or reduction of molecular oxygen, reduced iron-sulfur protein as one donor, and incorporation of one atom of oxygen [GO:0016713]